regulation of toll-like receptor 7 signaling pathway [GO:0034155] (biological process) Also known as: regulation of TLR7 signaling pathway, regulation of toll-like receptor 7 signalling pathway Definition: Any process that modulates the frequency, rate, or extent of toll-like receptor 7 signaling pathway. Subtypes: GO:0034156, positive regulation of toll-like receptor 7 signaling pathway [GO:0034157] Relationships: is_a regulation of cytoplasmic pattern recognition receptor signaling pathway [GO:0039531]; regulates toll-like receptor 7 signaling pathway [GO:0034154] References: PMID:16551253, PMID:17328678 Sources: GOC:add